{
  "gene": "UniProtKB:Q14410",
  "term_label": "glycerol metabolic process",
  "gene_symbol": "GK2",
  "gene_name": "Glycerol kinase 2",
  "term_id": "GO:0006071"
}